{
  "gene": "UniProtKB:Q9UK73",
  "term_id": "GO:0000151",
  "gene_symbol": "FEM1B",
  "term_label": "ubiquitin ligase complex",
  "gene_name": "Protein fem-1 homolog B"
}